{
  "gene_name": "ATP-dependent RNA helicase DDX25",
  "term_label": "mRNA binding",
  "term_id": "GO:0003729",
  "gene": "UniProtKB:Q9UHL0",
  "gene_symbol": "DDX25"
}